{
  "gene_name": "N-acyl-phosphatidylethanolamine-hydrolyzing phospholipase D",
  "gene_symbol": "NAPEPLD",
  "term_label": "N-acylethanolamine metabolic process",
  "term_id": "GO:0070291",
  "gene": "UniProtKB:Q6IQ20"
}